{
  "gene": "UniProtKB:Q96JB1",
  "gene_name": "Dynein axonemal heavy chain 8",
  "term_id": "GO:0036126",
  "gene_symbol": "DNAH8",
  "term_label": "sperm flagellum"
}